{
  "term_label": "guanyl-nucleotide exchange factor activity",
  "gene_name": "Vacuolar fusion protein MON1 homolog B",
  "gene": "UniProtKB:Q7L1V2",
  "gene_symbol": "MON1B",
  "term_id": "GO:0005085"
}